{
  "term_id": "UNKNOWN:0002",
  "gene_name": "U5 small nuclear ribonucleoprotein 40 kDa protein",
  "term_label": "Unknown biological process",
  "gene_symbol": "SNRNP40",
  "gene": "UniProtKB:Q96DI7"
}